hypoglossal nerve maturation [GO:0021619] (biological process) Definition: A developmental process, independent of morphogenetic (shape) change, that is required for the hypoglossal nerve to attain its fully functional state. This motor nerve innervates all the intrinsic and all but one of the extrinsic muscles of the tongue. Sources: GOC:cls, GOC:dgh, GOC:dph, GOC:jid, GO_REF:0000021 Relationships: is a type of GO:0021605; is part of hypoglossal nerve development [GO:0021566] Also known as: CN XII maturation